{
  "gene_symbol": "H2BC5",
  "gene": "UniProtKB:P58876",
  "gene_name": "Histone H2B type 1-D",
  "term_id": "GO:0006325",
  "term_label": "chromatin organization"
}